3,9-dihydroxypterocarpan 6a-monooxygenase activity [GO:0047082] (molecular function) Relationships: is a type of GO:0016709 Sources: EC:1.14.14.93, RHEA:15321 Also known as: 3,9-dihydroxypterocarpan 6a-hydroxylase activity, (6aR,11aR)-3,9-dihydroxypterocarpan,NADPH:oxygen oxidoreductase (6a-hydroxylating), 3,9-dihydroxypterocarpan 6alpha-monooxygenase Definition: Catalysis of the reaction: (6aR,11aR)-3,9-dihydroxypterocarpan + H+ + NADPH + O2 = (6aS,11aS)-3,6a,9-trihydroxypterocarpan + H2O + NADP+. (6aS,11aS)-3,6a,9-trihydroxypterocarpan is also known as (-)-glycinol.